{
  "term_id": "GO:0005634",
  "term_label": "nucleus",
  "gene_name": "Rac GTPase-activating protein 1",
  "gene": "UniProtKB:Q9H0H5",
  "gene_symbol": "RACGAP1"
}